trachea development [GO:0060438] (biological process) Relationships: is a type of animal organ development [GO:0048513]; is part of respiratory system development [GO:0060541] Sources: GOC:dph Definition: The process whose specific outcome is the progression of a trachea over time, from its formation to the mature structure. The trachea is the portion of the airway that attaches to the bronchi as it branches.